{
  "gene_name": "Tropomodulin-2",
  "term_id": "GO:0005856",
  "term_label": "cytoskeleton",
  "gene": "UniProtKB:Q9NZR1",
  "gene_symbol": "TMOD2"
}